{
  "gene": "UniProtKB:P17813",
  "term_id": "UNKNOWN:0001",
  "gene_symbol": "ENG",
  "term_label": "Unknown molecular function",
  "gene_name": "Endoglin"
}